dibutyl phthalate binding [GO:0035275] (molecular function) Relationships: is_a binding [GO:0005488] Definition: Binding to dibutyl phthalate, C(16)H(22)O(4). References: PMID:31954361, PMID:35408690 Also known as: DBP binding, phthalic acid dibutyl ester binding